{
  "term_label": "ubiquitin binding",
  "gene_symbol": "NBR1",
  "gene_name": "Next to BRCA1 gene 1 protein",
  "gene": "UniProtKB:Q14596",
  "term_id": "GO:0043130"
}